{
  "term_label": "chaperone-mediated protein complex assembly",
  "gene_symbol": "BBS12",
  "gene": "UniProtKB:Q6ZW61",
  "term_id": "GO:0051131",
  "gene_name": "Bardet-Biedl syndrome 12 protein"
}